{
  "term_id": "GO:0016192",
  "gene": "UniProtKB:O60333",
  "gene_name": "Kinesin-like protein KIF1B",
  "term_label": "vesicle-mediated transport",
  "gene_symbol": "KIF1B"
}